{
  "term_id": "GO:0006954",
  "gene_name": "Interleukin-8",
  "gene": "UniProtKB:P10145",
  "gene_symbol": "CXCL8",
  "term_label": "inflammatory response"
}